{
  "term_id": "GO:0006357",
  "term_label": "regulation of transcription by RNA polymerase II",
  "gene_name": "Zinc finger protein 343",
  "gene_symbol": "ZNF343",
  "gene": "UniProtKB:Q6P1L6"
}